{
  "term_id": "GO:0035591",
  "gene": "UniProtKB:Q9BXL6",
  "term_label": "signaling adaptor activity",
  "gene_name": "Caspase recruitment domain-containing protein 14",
  "gene_symbol": "CARD14"
}